{
  "gene_name": "ATPase PAAT",
  "gene": "UniProtKB:Q9H8K7",
  "term_id": "GO:0016887",
  "gene_symbol": "PAAT",
  "term_label": "ATP hydrolysis activity"
}